cell junction assembly [GO:0034329] (biological process) Relationships: is a type of cellular component assembly [GO:0022607]; is a type of cell junction organization [GO:0034330] Definition: A cellular process that results in the aggregation, arrangement and bonding together of a set of components to form a cell junction. Sources: GOC:mah Regulation: regulated by regulation of cell junction assembly [GO:1901888]; negatively regulated by negative regulation of cell junction assembly [GO:1901889]; positively regulated by positive regulation of cell junction assembly [GO:1901890] Subtypes: cell-cell junction assembly [GO:0007043], cell-substrate junction assembly [GO:0007044], synapse assembly [GO:0007416]